{
  "gene_symbol": "ACBD4",
  "gene": "UniProtKB:Q8NC06",
  "term_label": "fatty-acyl-CoA binding",
  "term_id": "GO:0000062",
  "gene_name": "Acyl-CoA-binding domain-containing protein 4"
}